{
  "term_id": "UNKNOWN:0003",
  "gene": "UniProtKB:Q9UGK3",
  "term_label": "Unknown cellular component",
  "gene_symbol": "STAP2",
  "gene_name": "Signal-transducing adaptor protein 2"
}